{
  "term_label": "vesicle-mediated transport",
  "gene": "UniProtKB:P61018",
  "gene_name": "Ras-related protein Rab-4B",
  "gene_symbol": "RAB4B",
  "term_id": "GO:0016192"
}